cyclic nucleotide phosphodiesterase activator activity [GO:0170005] (molecular function) Definition: Binds to and increases the activity of cyclic nucleotide phosphodiesterase. References: PMID:6087882, PMID:6259174, PMID:6667031 Relationships: is a type of GO:0008047; positively regulates cyclic-nucleotide phosphodiesterase activity [GO:0004112]